{
  "term_label": "DNA replication, synthesis of primer",
  "gene_name": "DNA primase small subunit",
  "gene_symbol": "PRIM1",
  "term_id": "GO:0006269",
  "gene": "UniProtKB:P49642"
}